{
  "term_label": "regulation of RNA splicing",
  "gene": "UniProtKB:Q9BXM0",
  "term_id": "GO:0043484",
  "gene_name": "Periaxin",
  "gene_symbol": "PRX"
}